positive regulation of somitomeric trunk muscle development [GO:0014709] (biological process) Sources: GOC:mtg_muscle Definition: Any process that activates, maintains or increases the frequency, rate or extent of somitomeric trunk muscle development. The somitomeric trunk muscle is derived from somitomeric mesoderm. The muscle begins its development with the differentiation of the muscle cells and ends with the mature muscle. Relationships: is a type of regulation of somitomeric trunk muscle development [GO:0014708]; is a type of positive regulation of muscle organ development [GO:0048636]; RO_0002213 GO:0002075